{
  "gene_symbol": "LRRC8D",
  "gene": "UniProtKB:Q7L1W4",
  "term_id": "GO:0005225",
  "gene_name": "Volume-regulated anion channel subunit LRRC8D",
  "term_label": "volume-sensitive anion channel activity"
}